{
  "term_id": "GO:0015645",
  "term_label": "fatty acid ligase activity",
  "gene_symbol": "ACSM5",
  "gene_name": "Acyl-coenzyme A synthetase ACSM5, mitochondrial",
  "gene": "UniProtKB:Q6NUN0"
}